{
  "term_label": "Unknown cellular component",
  "term_id": "UNKNOWN:0003",
  "gene_symbol": "CCDC192",
  "gene_name": "Coiled-coil domain-containing protein 192",
  "gene": "UniProtKB:P0DO97"
}